{
  "term_label": "Unknown molecular function",
  "gene": "UniProtKB:V9GZ13",
  "term_id": "UNKNOWN:0001",
  "gene_name": "MKKS centrosomal shuttling protein",
  "gene_symbol": "MKKS"
}